benzoate metabolic process [GO:0018874] (biological process) Definition: The chemical reactions and pathways involving benzoate, the anion of benzoic acid (benzenecarboxylic acid), a fungistatic compound widely used as a food preservative; it is conjugated to glycine in the liver and excreted as hippuric acid. Sources: ISBN:0721662544 Also known as: benzoate metabolism Relationships: is a type of monocarboxylic acid metabolic process [GO:0032787]; is a type of benzene-containing compound metabolic process [GO:0042537] Subtypes: (R)-mandelate catabolic process to benzoate [GO:0019597], benzoate catabolic process [GO:0043639]